{
  "gene": "UniProtKB:P78381",
  "gene_symbol": "SLC35A2",
  "gene_name": "UDP-galactose translocator",
  "term_label": "UDP-galactose transmembrane transporter activity",
  "term_id": "GO:0005459"
}